{
  "gene": "UniProtKB:P25705",
  "term_id": "GO:0005524",
  "gene_symbol": "ATP5F1A",
  "term_label": "ATP binding",
  "gene_name": "ATP synthase subunit alpha, mitochondrial"
}